{
  "gene": "UniProtKB:P47985",
  "term_id": "GO:0045275",
  "gene_name": "Cytochrome b-c1 complex subunit Rieske, mitochondrial",
  "term_label": "respiratory chain complex III",
  "gene_symbol": "UQCRFS1"
}